{
  "gene_name": "Putative solute carrier organic anion transporter family member 1B7",
  "gene": "UniProtKB:G3V0H7",
  "gene_symbol": "SLCO1B7",
  "term_id": "GO:0015125",
  "term_label": "bile acid transmembrane transporter activity"
}